{
  "gene_symbol": "PRODH",
  "term_id": "GO:0005739",
  "term_label": "mitochondrion",
  "gene_name": "Proline dehydrogenase 1, mitochondrial",
  "gene": "UniProtKB:O43272"
}